{
  "term_id": "GO:0007155",
  "gene_symbol": "SIGLEC12",
  "gene": "UniProtKB:Q96PQ1",
  "gene_name": "Sialic acid-binding Ig-like lectin 12",
  "term_label": "cell adhesion"
}